{
  "term_id": "GO:0000226",
  "term_label": "microtubule cytoskeleton organization",
  "gene": "UniProtKB:O00423",
  "gene_name": "Echinoderm microtubule-associated protein-like 1",
  "gene_symbol": "EML1"
}